{
  "gene_name": "Megakaryocyte and platelet inhibitory receptor G6b",
  "term_label": "platelet formation",
  "gene": "UniProtKB:O95866",
  "term_id": "GO:0030220",
  "gene_symbol": "MPIG6B"
}